{
  "gene_name": "Torsin-1A",
  "term_label": "kinesin binding",
  "gene": "UniProtKB:O14656",
  "term_id": "GO:0019894",
  "gene_symbol": "TOR1A"
}